{
  "gene_name": "Adipose-secreted signaling protein",
  "term_id": "UNKNOWN:0003",
  "gene": "UniProtKB:Q9GZN8",
  "term_label": "Unknown cellular component",
  "gene_symbol": "ADISSP"
}